{
  "term_label": "Unknown cellular component",
  "gene_symbol": "NRK",
  "gene": "UniProtKB:Q7Z2Y5",
  "term_id": "UNKNOWN:0003",
  "gene_name": "Nik-related protein kinase"
}